Glc2Man9GlcNAc2 oligosaccharide glucosidase activity [GO:0106407] (molecular function) Relationships: is a type of alpha-glucosidase activity [GO:0090599] Definition: Catalysis of the reaction: Glc(2)Man(9)GlcNAc(2)-[protein] + H2O = GlcMan(9)GlcNAc(2)-[protein] + beta-D-glucopyranose. Note: Trims Glc alpha 1,3 Glc bond in Glc2Man9GlcNAc2 oligosaccharide in inmature glycoproteins. Also known as: glucosidase II References: PMID:30389790 Sources: EC:3.2.1.207